glycosylphosphatidylinositol-mannosyltransferase I complex [GO:1990529] (cellular component) Relationships: is a type of mannosyltransferase complex [GO:0031501]; is a type of endoplasmic reticulum protein-containing complex [GO:0140534] Definition: A protein complex that is involved in the transfer of the four mannoses in the GPI-anchor precursor. In yeast S. cerevisiae this complex consists of Pbn1p and Gpi14p and in rat this complex consists of PIG-X and PIG-M. Also known as: GPI-MT-I complex References: PMID:15635094 Sources: GOC:dph, GOC:rb